raffinose family oligosaccharide biosynthetic process [GO:0010325] (biological process) Definition: The chemical reactions and pathways resulting in the formation of raffinose family oligosaccharides (RFOs, such as raffinose, stachyose, verbascose and other molecules with a higher degree of galactosyl polymerization). Subtypes: raffinose biosynthetic process [GO:0033529], stachyose biosynthetic process [GO:0033532], GO:0033534, ajugose biosynthetic process [GO:0033536] Also known as: raffinose family oligosaccharide biosynthesis Sources: GOC:tair_curators Relationships: is a type of oligosaccharide biosynthetic process [GO:0009312]